regulation of glycine import across plasma membrane [GO:1900923] (biological process) Definition: Any process that modulates the frequency, rate or extent of glycine import into a cell. Sources: GOC:TermGenie Also known as: regulation of glycine import Relationships: is a type of regulation of amino acid import across plasma membrane [GO:0010958]; is a type of regulation of organic acid transport [GO:0032890]; regulates glycine import across plasma membrane [GO:1903804] Subtypes: negative regulation of glycine import across plasma membrane [GO:1900924], GO:1900925